cellular response to sterol [GO:0036315] (BP) Definition: Any process that results in a change in state or activity of a cell (in terms of movement, secretion, enzyme production, gene expression, etc.) as a result of a sterol stimulus. Relationships: is_a GO:0036314; is a type of cellular response to lipid [GO:0071396]; is a type of cellular response to oxygen-containing compound [GO:1901701] Sources: GOC:bf Subtypes: cellular response to ecdysone [GO:0071390], GO:0071397, cellular response to ergosterol [GO:1901625], cellular response to diosgenin [GO:1905093]